{
  "term_id": "GO:0016323",
  "gene": "UniProtKB:Q14542",
  "term_label": "basolateral plasma membrane",
  "gene_symbol": "SLC29A2",
  "gene_name": "Equilibrative nucleoside transporter 2"
}